{
  "term_id": "UNKNOWN:0003",
  "gene_symbol": "LINC00474",
  "gene": "UniProtKB:Q9P2X8",
  "term_label": "Unknown cellular component",
  "gene_name": "Putative uncharacterized protein encoded by LINC00474"
}